regulation of ethylene-activated signaling pathway [GO:0010104] (biological process) Definition: Any process that modulates the frequency, rate or extent of ethylene (ethene) signal transduction. Relationships: is a type of regulation of phosphorelay signal transduction system [GO:0070297]; regulates ethylene-activated signaling pathway [GO:0009873] Subtypes: negative regulation of ethylene-activated signaling pathway [GO:0010105] Sources: GOC:tb Also known as: regulation of ethene mediated signaling pathway, regulation of ethene mediated signalling pathway, regulation of ethylene mediated signalling pathway, regulation of ethylene mediated signaling pathway